{
  "gene_name": "Meiotic nuclear division protein 1 homolog",
  "term_label": "Unknown molecular function",
  "term_id": "UNKNOWN:0001",
  "gene_symbol": "MND1",
  "gene": "UniProtKB:Q9BWT6"
}